cell proliferation involved in neural plate elongation [GO:0021992] (biological process) Definition: The process of expansion of cell numbers in the neural plate due to cell division of progenitor cells preferentially in the rostrocaudal direction, resulting in the elongation of the tissue. Relationships: is a type of GO:0061351; is part of neural plate elongation [GO:0014022] References: PMID:15806586 Sources: GOC:cls, GOC:dgh, GOC:dph, GOC:jid, GO_REF:0000021